{
  "gene_symbol": "UBE2B",
  "gene": "UniProtKB:P63146",
  "term_id": "GO:0033503",
  "term_label": "HULC complex",
  "gene_name": "Ubiquitin-conjugating enzyme E2 B"
}